ciliary basal body [GO:0036064] (cellular component) Definition: A membrane-tethered, short cylindrical array of microtubules and associated proteins found at the base of a eukaryotic cilium (also called flagellum) that is similar in structure to a centriole and derives from it. The cilium basal body is the site of assembly and remodeling of the cilium and serves as a nucleation site for axoneme growth. As well as anchoring the cilium, it is thought to provide a selective gateway regulating the entry of ciliary proteins and vesicles by intraflagellar transport. Note: In most eukaryotic cells, 'ciliary basal body' (GO:0036064) and 'centriole' (GO:0005814) represent a common entity that cycles through its function in cell division, then ciliogenesis, then cell division again. However, these structures are modified extensively as they transition into each other, and may contain different proteins, specific to each component. Subtypes: kinociliary basal body [GO:1902636], GO:1902671, GO:1902672, GO:1902673, right posteriolateral basal body [GO:1902674], left ventral basal body [GO:1902675], right ventral basal body [GO:1902676], left caudal basal body [GO:1902677], GO:1902678 Also known as: basal body, cilial basal body, cilium basal body, kinetosome, microtubule basal body References: PMID:21750193 Sources: GOC:cilia, GOC:clt Relationships: is a type of microtubule organizing center [GO:0005815]; is part of GO:0005929